{
  "term_id": "GO:0019905",
  "gene_symbol": "STXBP4",
  "term_label": "syntaxin binding",
  "gene": "UniProtKB:Q6ZWJ1",
  "gene_name": "Syntaxin-binding protein 4"
}